3-methylquercetin 3'-O-methyltransferase activity [GO:0102445] (molecular function) Relationships: is a type of methyltransferase activity [GO:0008168] Sources: RHEA:74715 Definition: Catalysis of the reaction: 3',4',5,7-tetrahydroxy-3-methoxyflavone + S-adenosyl-L-methionine = 3,3'-O-dimethylquercetin + H+ + S-adenosyl-L-homocysteine.